{
  "term_id": "UNKNOWN:0003",
  "gene_name": "Immunoglobulin heavy variable 4_OR15-8 (non-functional) (Fragment)",
  "term_label": "Unknown cellular component",
  "gene_symbol": "IGHV4OR15-8",
  "gene": "UniProtKB:A0A075B7B6"
}